{
  "gene_symbol": "KIAA1671",
  "gene": "UniProtKB:Q9BY89",
  "term_label": "Unknown molecular function",
  "gene_name": "Uncharacterized protein KIAA1671",
  "term_id": "UNKNOWN:0001"
}